{
  "gene_name": "cGMP-dependent 3',5'-cyclic phosphodiesterase",
  "gene_symbol": "PDE2A",
  "term_id": "GO:0042803",
  "gene": "UniProtKB:O00408",
  "term_label": "protein homodimerization activity"
}